lipid droplet fusion [GO:0160077] (biological process) Relationships: is a type of lipid droplet organization [GO:0034389]; is a type of GO:0048284 Regulation: negatively regulated by negative regulation of lipid droplet fusion [GO:0160078] Definition: The process by which a single lipid droplet is created from the fusion of two or more lipid droplets. References: PMID:34508658, PMID:36477540